{
  "term_id": "GO:0016486",
  "gene": "UniProtKB:P29120",
  "term_label": "peptide hormone processing",
  "gene_symbol": "PCSK1",
  "gene_name": "Neuroendocrine convertase 1"
}